basement membrane organization [GO:0071711] (biological process) Definition: A process that is carried out at the cellular level which results in the assembly, arrangement of constituent parts, or disassembly of the basement membrane. Also known as: basement membrane organisation Regulation: regulated by GO:0110011 Relationships: is a type of extracellular matrix organization [GO:0030198] Subtypes: basement membrane disassembly [GO:0034769], basement membrane assembly [GO:0070831] Sources: GOC:mah Note: Note that this term has no relationship to 'membrane organization ; GO:0061024' because the basement membrane is not a lipid bilayer.